phosphatidylcholine biosynthesis from sn-glycero-3-phosphocholine [GO:0090640] (biological process) References: PMID:24329598, PMID:27758859 Sources: MetaCyc:PWY-7470 Definition: The phosphatidylcholine biosynthetic process that involves the two-step acylation of sn-glycero-3-phosphocholine to a phosphatidylcholine. Relationships: is_a phosphatidylcholine biosynthetic process [GO:0006656]